{
  "term_label": "plasma membrane",
  "term_id": "GO:0005886",
  "gene": "UniProtKB:Q13191",
  "gene_name": "E3 ubiquitin-protein ligase CBL-B",
  "gene_symbol": "CBLB"
}